{
  "gene_name": "[Pyruvate dehydrogenase (acetyl-transferring)] kinase isozyme 2, mitochondrial",
  "term_label": "mitochondrion",
  "gene_symbol": "PDK2",
  "term_id": "GO:0005739",
  "gene": "UniProtKB:Q15119"
}